regulation of spore germination [GO:1904359] (biological process) References: PMID:14718564, PMID:8798577 Sources: GOC:TermGenie, GO_REF:0000058 Also known as: modulation of spore germination on or near host Subtypes: regulation of encysted zoospore germination [GO:0075227], negative regulation of spore germination [GO:1904360], GO:1904361 Relationships: is a type of regulation of developmental process [GO:0050793]; is_a regulation of cellular process [GO:0050794]; RO_0002211 GO:0009847 Definition: Any process that modulates the frequency, rate or extent of spore germination.